pre-miRNA export from nucleus [GO:0035281] (BP) References: PMID:14744438 Sources: GOC:sl Also known as: pre-microRNA export from cell nucleus, pre-microRNA export out of nucleus, pre-microRNA transport from nucleus to cytoplasm, pre-microRNA-nucleus export, pre-microRNA export from nucleus Relationships: is_a GO:0006405; BFO_0000050 miRNA-mediated post-transcriptional gene silencing [GO:0035195] Definition: Transport of pre-microRNAs (pre-miRNAs) from the nucleus to the cytoplasm. Pre-miRNAs are a ~60-70 nucleotide stem loop intermediate in miRNA production, produced by the nuclear cleavage of a primary miRNA (pri-mRNA) transcript. Pre-miRNAs are transported from the nucleus to the cytoplasm where further cleavage occurs to produce a mature miRNA product.